{
  "term_id": "GO:0003723",
  "term_label": "RNA binding",
  "gene_name": "U6 snRNA-associated Sm-like protein LSm3",
  "gene_symbol": "LSM3",
  "gene": "UniProtKB:P62310"
}